{
  "gene": "UniProtKB:Q13761",
  "term_label": "hemopoiesis",
  "gene_name": "Runt-related transcription factor 3",
  "gene_symbol": "RUNX3",
  "term_id": "GO:0030097"
}